{
  "term_label": "Unknown cellular component",
  "gene_name": "Cortexin-2",
  "term_id": "UNKNOWN:0003",
  "gene": "UniProtKB:P0C2S0",
  "gene_symbol": "CTXN2"
}